{
  "term_label": "protein kinase inhibitor activity",
  "term_id": "GO:0004860",
  "gene_symbol": "PAK1IP1",
  "gene": "UniProtKB:Q9NWT1",
  "gene_name": "p21-activated protein kinase-interacting protein 1"
}